{
  "gene_name": "6-phosphofructo-2-kinase_fructose-2,6-bisphosphatase 3",
  "term_label": "fructose-2,6-bisphosphate 2-phosphatase activity",
  "gene": "UniProtKB:Q16875",
  "term_id": "GO:0004331",
  "gene_symbol": "PFKFB3"
}